{
  "gene_symbol": "NAGLU",
  "term_id": "GO:0005773",
  "gene": "UniProtKB:P54802",
  "gene_name": "Alpha-N-acetylglucosaminidase",
  "term_label": "vacuole"
}